{
  "gene_symbol": "FBXL18",
  "term_id": "UNKNOWN:0001",
  "gene": "UniProtKB:Q96ME1",
  "gene_name": "F-box_LRR-repeat protein 18",
  "term_label": "Unknown molecular function"
}